histone H2AS1 kinase activity [GO:0044024] (molecular function) Definition: Catalysis of the reaction: histone H2A-serine (position 1) + ATP = histone H2A-phosphoserine (position 1) + ADP. This reaction is the addition of a phosphate group to the serine residue at position 1 of histone H2A. Relationships: is a type of protein serine/threonine kinase activity [GO:0004674]; is a type of histone H2A kinase activity [GO:0140995] Also known as: histone kinase activity (H2A-S1 specific), histone serine kinase activity (H2A-S1 specific), histone-serine kinase activity (H2A-S1 specific) Note: Note that the residue position corresponds to the canonical human H2A2A histone (UniProtKB:Q6FI13); this residue is conserved across all eukaryotes, but missing from Drosophila histone H2AV. Residue 1 is the first residue following removal of the initiating Methionine (Met). Note that each histone is encoded by multiple genes, and sequences may vary across different genes within an organism. Sources: GOC:jl